(1->3),(1->4)-beta-glucan binding [GO:2001077] (molecular function) Also known as: (1,3),(1,4)-beta-glucan binding, 1->3,1->4-beta-glucan binding, beta-(1,3),(1,4)-glucan binding, beta-(1->3),(1->4)-glucan binding, beta-1,3-1,4-glucan binding, beta-1->3,1->4-glucan binding Relationships: is a type of GO:0030247 Definition: Binding to (1->3),(1->4)-beta-glucan. Sources: GOC:mengo_curators